positive regulation of tendon cell differentiation [GO:2001051] (biological process) Definition: Any process that activates or increases the frequency, rate or extent of tendon cell differentiation. Also known as: positive regulation of muscle attachment cell differentiation, positive regulation of tenocyte differentiation Sources: GOC:obol Relationships: is a type of GO:0045597; is a type of GO:2001049; RO_0002213 tendon cell differentiation [GO:0035990]